negative regulation of lysosomal protein catabolic process [GO:1905166] (biological process) Also known as: down regulation of cellular protein breakdown in lysosome, down regulation of cellular protein catabolic process in lysosome, down regulation of cellular protein catabolism in lysosome, down regulation of cellular protein degradation in lysosome, down regulation of lysosomal protein catabolic process, down regulation of lysosomal protein catabolism, down regulation of lysosomal protein degradation, down-regulation of cellular protein breakdown in lysosome, down-regulation of cellular protein catabolic process in lysosome, down-regulation of cellular protein catabolism in lysosome, down-regulation of cellular protein degradation in lysosome, down-regulation of lysosomal protein catabolic process, down-regulation of lysosomal protein catabolism, down-regulation of lysosomal protein degradation, downregulation of cellular protein breakdown in lysosome, downregulation of cellular protein catabolic process in lysosome, downregulation of cellular protein catabolism in lysosome, downregulation of cellular protein degradation in lysosome, downregulation of lysosomal protein catabolic process, downregulation of lysosomal protein catabolism, downregulation of lysosomal protein degradation, negative regulation of cellular protein breakdown in lysosome, negative regulation of cellular protein catabolic process in lysosome, negative regulation of cellular protein catabolism in lysosome, negative regulation of cellular protein degradation in lysosome, negative regulation of lysosomal protein catabolism, negative regulation of lysosomal protein degradation, inhibition of cellular protein breakdown in lysosome, inhibition of cellular protein catabolic process in lysosome, inhibition of cellular protein catabolism in lysosome, inhibition of cellular protein degradation in lysosome, inhibition of lysosomal protein catabolic process, inhibition of lysosomal protein catabolism, inhibition of lysosomal protein degradation, down regulation of lysosomal proteolysis, down regulation of proteolysis within lysosome, down-regulation of lysosomal proteolysis, down-regulation of proteolysis within lysosome, downregulation of lysosomal proteolysis, downregulation of proteolysis within lysosome, inhibition of lysosomal proteolysis, inhibition of proteolysis within lysosome, negative regulation of lysosomal proteolysis, negative regulation of proteolysis within lysosome Relationships: is_a negative regulation of protein catabolic process in the vacuole [GO:1904351]; is a type of regulation of lysosomal protein catabolic process [GO:1905165]; negatively regulates lysosomal protein catabolic process [GO:1905146] Sources: GOC:PARL, GOC:TermGenie, GOC:bf, GO_REF:0000058 Definition: Any process that stops, prevents or reduces the frequency, rate or extent of lysosomal protein catabolic process.